delta(3,5)-delta(2,4)-dienoyl-CoA isomerase activity [GO:0051750] (molecular function) Definition: Catalysis of the reaction: a (3E,5Z)-dienoyl-CoA = a (2E,4E)-(5,6-saturated)-dienoyl-CoA. Relationships: is a type of intramolecular oxidoreductase activity, transposing C=C bonds [GO:0016863] References: PMID:11278886, PMID:16040662 Sources: RHEA:45240 Also known as: delta(3,5),delta(2,4)-dienoyl-coenzyme A isomerase activity, delta3,5-delta2,4-dienoyl-CoA isomerase activity, delta5-delta2,4-dienoyl-CoA isomerase activity